{
  "gene": "UniProtKB:Q15111",
  "term_id": "UNKNOWN:0003",
  "gene_symbol": "PLCL1",
  "term_label": "Unknown cellular component",
  "gene_name": "Inactive phospholipase C-like protein 1"
}